{
  "term_id": "GO:0003735",
  "gene_name": "Large ribosomal subunit protein uL11m",
  "gene_symbol": "MRPL11",
  "term_label": "structural constituent of ribosome",
  "gene": "UniProtKB:Q9Y3B7"
}